positive regulation of smooth muscle contraction [GO:0045987] (biological process) Definition: Any process that activates or increases the frequency, rate or extent of smooth muscle contraction. Subtypes: positive regulation of hindgut contraction [GO:0060450], positive regulation of uterine smooth muscle contraction [GO:0070474], positive regulation of gastro-intestinal system smooth muscle contraction [GO:1904306], positive regulation of smooth muscle contraction involved in micturition [GO:1904320], positive regulation of vascular associated smooth muscle contraction [GO:1904695] Also known as: up regulation of smooth muscle contraction, up-regulation of smooth muscle contraction, upregulation of smooth muscle contraction, activation of smooth muscle contraction, stimulation of smooth muscle contraction Relationships: is a type of regulation of smooth muscle contraction [GO:0006940]; is a type of positive regulation of muscle contraction [GO:0045933]; RO_0002213 smooth muscle contraction [GO:0006939] Sources: GOC:go_curators